anaerobic carbon-monoxide dehydrogenase activity [GO:0043885] (MF) Sources: RHEA:21040 Also known as: carbon monoxide dehydrogenase activity, carbon-monoxide dehydrogenase activity, CO dehydrogenase activity, CO-dehydrogenase (ferredoxin) activity, CO-dehydrogenase activity, carbon monoxide dehydrogenase (ferredoxin) activity, carbon-monoxide dehydrogenase (ferredoxin) activity, carbon-monoxide,water:ferredoxin oxidoreductase activity, carbon-monoxide:(acceptor) oxidoreductase activity, CODH Definition: Catalysis of the reaction: CO + H2O + oxidized ferredoxin = CO2 + reduced ferredoxin. Relationships: is a type of oxidoreductase activity, acting on the aldehyde or oxo group of donors, iron-sulfur protein as acceptor [GO:0016625]